{
  "gene_name": "Probable G-protein coupled receptor 174",
  "term_id": "GO:0004930",
  "term_label": "G protein-coupled receptor activity",
  "gene": "UniProtKB:Q9BXC1",
  "gene_symbol": "GPR174"
}